{
  "gene": "UniProtKB:Q8WVF2",
  "gene_symbol": "UCMA",
  "gene_name": "Unique cartilage matrix-associated protein",
  "term_label": "extracellular matrix",
  "term_id": "GO:0031012"
}